{
  "term_label": "signal transduction",
  "gene_name": "Olfactory receptor 1F1",
  "gene_symbol": "OR1F1",
  "gene": "UniProtKB:O43749",
  "term_id": "GO:0007165"
}